{
  "term_id": "UNKNOWN:0003",
  "term_label": "Unknown cellular component",
  "gene": "UniProtKB:Q6P4F1",
  "gene_name": "Alpha-(1,3)-fucosyltransferase 10",
  "gene_symbol": "FUT10"
}